chylomicron binding [GO:0035478] (molecular function) Definition: Binding to a chylomicron, a large lipoprotein particle (diameter 75-1200 nm) composed of a central core of triglycerides and cholesterol surrounded by a protein-phospholipid coating. The proteins include one molecule of apolipoprotein B-48 and may include a variety of apolipoproteins, including APOAs, APOCs and APOE. References: PMID:17403372 Sources: GOC:BHF Relationships: is a type of GO:0071813